{
  "term_id": "GO:0071011",
  "gene_symbol": "SNRPD3",
  "term_label": "precatalytic spliceosome",
  "gene": "UniProtKB:P62318",
  "gene_name": "Small nuclear ribonucleoprotein Sm D3"
}